adenylosuccinate synthase activity [GO:0004019] (molecular function) Also known as: IMP--aspartate ligase activity, IMP:L-aspartate ligase (GDP-forming), adenylosuccinate synthetase activity, succino-AMP synthetase activity, succinoadenylic kinosynthetase activity Definition: Catalysis of the reaction: L-aspartate + GTP + IMP = N(6)-(1,2-dicarboxyethyl)-AMP + GDP + 3 H+ + phosphate. Sources: EC:6.3.4.4, RHEA:15753 Relationships: is_a GO:0016879